{
  "gene_name": "Paralemmin-3",
  "term_id": "UNKNOWN:0003",
  "gene_symbol": "PALM3",
  "term_label": "Unknown cellular component",
  "gene": "UniProtKB:A6NDB9"
}